{
  "gene": "UniProtKB:P37058",
  "term_label": "testosterone dehydrogenase (NADP+) activity",
  "gene_symbol": "HSD17B3",
  "term_id": "GO:0047045",
  "gene_name": "17-beta-hydroxysteroid dehydrogenase type 3"
}